regulation of hepatic stellate cell activation [GO:2000489] (BP) Relationships: is a type of regulation of cell activation [GO:0050865]; regulates GO:0035733 Subtypes: negative regulation of hepatic stellate cell activation [GO:2000490], positive regulation of hepatic stellate cell activation [GO:2000491] Sources: GOC:obol Definition: Any process that modulates the frequency, rate or extent of hepatic stellate cell activation.